axillary shoot meristem initiation [GO:0090506] (biological process) Definition: A developmental process that results in the initiation of an axillary shoot meristem. An axillary shoot meristem is a shoot meristem formed in the axil of a leaf. Sources: GOC:tb Relationships: is a type of meristem initiation [GO:0010014]; is part of secondary shoot formation [GO:0010223] Also known as: axillary bud meristem initiation